acrosome reaction [GO:0007340] (biological process) References: PMID:11175768, PMID:21042299, PMID:3886029 Sources: GOC:dph Note: If the release of the acrosome content occurs before the sperm reaches the zona pellucida, consider using premature acrosome loss. Definition: The discharge, by sperm, of a single, anterior secretory granule following the sperm's attachment to the zona pellucida of the oocyte. The process begins with the fusion of the outer acrosomal membrane with the sperm plasma membrane and ends with the exocytosis of the acrosomal contents into the zona pellucida. Relationships: is a type of reproductive process [GO:0022414]; is part of single fertilization [GO:0007338]; has part membrane fusion involved in acrosome reaction [GO:0002078]; has part acrosomal vesicle exocytosis [GO:0060478] Regulation: regulated by regulation of acrosome reaction [GO:0060046]; negatively regulated by negative regulation of acrosome reaction [GO:1902225]; positively regulated by positive regulation of acrosome reaction [GO:2000344]